{
  "gene_symbol": "HIF1A",
  "gene_name": "Hypoxia-inducible factor 1-alpha",
  "term_id": "GO:0071456",
  "term_label": "cellular response to hypoxia",
  "gene": "UniProtKB:Q16665"
}